{
  "gene_name": "Proteasome subunit alpha type-1",
  "gene_symbol": "PSMA1",
  "term_id": "GO:0043161",
  "term_label": "proteasome-mediated ubiquitin-dependent protein catabolic process",
  "gene": "UniProtKB:P25786"
}